[4Fe-4S] cluster assembly [GO:0044572] (biological process) Regulation: regulated by regulation of [4Fe-4S] cluster assembly [GO:1900491]; negatively regulated by negative regulation of [4Fe-4S] cluster assembly [GO:1900492]; positively regulated by positive regulation of [4Fe-4S] cluster assembly [GO:1900493] Relationships: is_a iron-sulfur cluster assembly [GO:0016226] Also known as: 4Fe-4S cluster assembly, [4Fe-4S] cluster biosynthetic process References: PMID:15952888 Sources: GOC:jl, GOC:mengo_curators, GOC:pde, GOC:tt, GOC:vw Definition: The incorporation of four iron atoms and four sulfur atoms into an iron-sulfur cluster.